{
  "term_id": "GO:0032956",
  "term_label": "regulation of actin cytoskeleton organization",
  "gene_symbol": "ARHGEF15",
  "gene": "UniProtKB:O94989",
  "gene_name": "Rho guanine nucleotide exchange factor 15"
}